{
  "gene_name": "Zinc finger and SCAN domain-containing protein 16",
  "term_label": "regulation of transcription by RNA polymerase II",
  "term_id": "GO:0006357",
  "gene_symbol": "ZSCAN16",
  "gene": "UniProtKB:Q9H4T2"
}